{
  "gene": "UniProtKB:Q15477",
  "term_id": "GO:0055087",
  "gene_name": "Superkiller complex protein 2",
  "term_label": "Ski complex",
  "gene_symbol": "SKIC2"
}